{
  "gene_symbol": "MAGEA6",
  "term_label": "histone deacetylase binding",
  "term_id": "GO:0042826",
  "gene_name": "Melanoma-associated antigen 6",
  "gene": "UniProtKB:P43360"
}